{
  "gene_symbol": "IFI27L2",
  "term_label": "intrinsic apoptotic signaling pathway",
  "term_id": "GO:0097193",
  "gene": "UniProtKB:Q9H2X8",
  "gene_name": "Interferon alpha-inducible protein 27-like protein 2"
}